{
  "gene_symbol": "MCRIP1",
  "gene_name": "Mapk-regulated corepressor-interacting protein 1",
  "gene": "UniProtKB:C9JLW8",
  "term_id": "UNKNOWN:0002",
  "term_label": "Unknown biological process"
}